fluconazole transport [GO:0015903] (biological process) Definition: The directed movement of fluconazole into, out of or within a cell, or between cells, by means of some agent such as a transporter or pore. Fluconazole is an antifungal drug used for oral candidiasis and cryptococcal meningitis; it is still under study for treatment of vaginal candidiasis and other fungal infections. Relationships: is a type of organic hydroxy compound transport [GO:0015850]; is a type of nitrogen compound transport [GO:0071705] Sources: GOC:curators